{
  "gene_symbol": "DNAH1",
  "term_id": "GO:0030317",
  "gene": "UniProtKB:Q9P2D7",
  "term_label": "flagellated sperm motility",
  "gene_name": "Dynein axonemal heavy chain 1"
}